{
  "term_id": "GO:0072518",
  "gene": "UniProtKB:O75116",
  "gene_symbol": "ROCK2",
  "term_label": "Rho-dependent protein serine/threonine kinase activity",
  "gene_name": "Rho-associated protein kinase 2"
}